{
  "term_id": "GO:0005886",
  "gene_symbol": "RND1",
  "term_label": "plasma membrane",
  "gene": "UniProtKB:Q92730",
  "gene_name": "Rho-related GTP-binding protein Rho6"
}